cspyrone B1 catabolic process [GO:1900801] (biological process) Sources: GOC:TermGenie, GOC:di Relationships: is a type of ketone catabolic process [GO:0042182]; is a type of carboxylic acid catabolic process [GO:0046395]; is a type of secondary metabolite catabolic process [GO:0090487]; is a type of lactone catabolic process [GO:1901335] Also known as: cspyrone B1 breakdown, cspyrone B1 catabolism, cspyrone B1 degradation Definition: The chemical reactions and pathways resulting in the breakdown of cspyrone B1.